{
  "gene_name": "Charged multivesicular body protein 4b",
  "term_label": "Unknown molecular function",
  "term_id": "UNKNOWN:0001",
  "gene": "UniProtKB:Q9H444",
  "gene_symbol": "CHMP4B"
}